{
  "gene": "UniProtKB:Q96PN7",
  "gene_symbol": "TRERF1",
  "term_label": "transcription regulator complex",
  "gene_name": "Transcriptional-regulating factor 1",
  "term_id": "GO:0005667"
}